DNA helicase A complex [GO:0033203] (CC) Relationships: is a type of DNA helicase complex [GO:0033202]; is_a GO:0140513 Definition: A homohexameric protein complex that possesses DNA helicase activity; associates with DNA polymerase alpha-primase and translocates in the 5' to 3' direction. References: PMID:9341218